alpha6-beta1 integrin-CYR61 complex [GO:0071116] (cellular component) Also known as: ITGA6-ITGB1-CYR61 complex Definition: A protein complex that consists of an alpha6-beta1 integrin complex bound to CYR61, a cysteine-rich protein involved in angiogenesis. References: PMID:12826661 Relationships: is a type of GO:0098797